viral budding from endoplasmic reticulum membrane [GO:0046762] (biological process) Sources: GOC:bf, GOC:jl, ISBN:0072370319, VZ:1947 Relationships: is a type of viral budding [GO:0046755] Definition: A viral budding that starts with formation of a membrane curvature in the host ER membrane. Also known as: ER membrane viral budding, endoplasmic reticulum membrane viral budding, viral budding from ER membrane, virus budding from ER membrane, virus budding from ER membrane by viral capsid envelopment, ER membrane viral budding during viral capsid envelopment, endoplasmic reticulum membrane viral budding during viral capsid envelopment, viral budding from ER membrane by viral capsid envelopment, viral budding from ER membrane during viral capsid envelopment, virus budding from ER membrane during viral capsid envelopment